regulation of reproductive process [GO:2000241] (biological process) Subtypes: adaptation to pheromone regulating conjugation with mutual genetic exchange [GO:0000760], regulation of flower development [GO:0009909], regulation of floral meristem growth [GO:0010080], GO:0010081, regulation of reciprocal meiotic recombination [GO:0010520], regulation of meiotic joint molecule formation [GO:0010946], regulation of conjugation with cellular fusion [GO:0031137], regulation of mating type switching [GO:0031494], regulation of fusion of sperm to egg plasma membrane [GO:0043012], GO:0045477, regulation of embryo sac egg cell differentiation [GO:0045694], regulation of egg-laying behavior [GO:0046662], regulation of male pigmentation [GO:0048088], regulation of female pigmentation [GO:0048089], regulation of meiotic cell cycle [GO:0051445], regulation of acrosome reaction [GO:0060046], regulation of ovulation [GO:0060278], regulation of penile erection [GO:0060405], regulation of ascospore wall beta-glucan biosynthetic process [GO:0060622], regulation of homologous chromosome segregation [GO:0060629], regulation of prostatic bud formation [GO:0060685], GO:0060687, regulation of cell differentiation involved in embryonic placenta development [GO:0060800], regulation of floral organ abscission [GO:0060860], regulation of premature acrosome loss [GO:0061949], GO:0070799, regulation of phialide development [GO:0070805], GO:0070808, regulation of spore-bearing organ development [GO:0075260], regulation of seed development [GO:0080050], GO:0080092, regulation of fertilization [GO:0080154], regulation of synaptonemal complex assembly [GO:0090173], regulation of anther dehiscence [GO:0120194], regulation of oocyte karyosome formation [GO:0120313], regulation of oocyte maturation [GO:1900193], regulation of flagellated sperm motility [GO:1901317], regulation of meiotic cell cycle phase transition [GO:1901993], regulation of meiotic spindle elongation [GO:1902119], regulation of male mating behavior [GO:1902435], regulation of sperm capacitation [GO:1902490], regulation of ascospore-type prospore membrane formation [GO:1903023], GO:1903341, regulation of meiotic cell cycle process involved in oocyte maturation [GO:1903538], GO:1903664, regulation of maternal process involved in parturition [GO:1904301], regulation of establishment of Sertoli cell barrier [GO:1904444], GO:1904967, regulation of meiotic chromosome separation [GO:1905132], regulation of amoeboid sperm motility [GO:1905416], regulation of oogenesis [GO:1905879], GO:1905939, regulation of endosperm development [GO:2000014], GO:2000242, GO:2000243, regulation of FtsZ-dependent cytokinesis [GO:2000244], regulation of antral ovarian follicle growth [GO:2000387] Relationships: is a type of regulation of biological process [GO:0050789]; regulates reproductive process [GO:0022414] Sources: GOC:mah Definition: Any process that modulates the frequency, rate or extent of reproductive process.